{
  "gene": "UniProtKB:Q9UBC5",
  "term_label": "actin filament-based movement",
  "gene_symbol": "MYO1A",
  "term_id": "GO:0030048",
  "gene_name": "Unconventional myosin-Ia"
}